{
  "gene": "UniProtKB:Q15937",
  "gene_symbol": "ZNF79",
  "term_id": "GO:0006357",
  "gene_name": "Zinc finger protein 79",
  "term_label": "regulation of transcription by RNA polymerase II"
}